{
  "gene": "UniProtKB:P35658",
  "gene_name": "Nuclear pore complex protein Nup214",
  "term_label": "protein import into nucleus",
  "gene_symbol": "NUP214",
  "term_id": "GO:0006606"
}